fraxetin 5-hydroxylase activity [GO:0106144] (molecular function) Definition: Catalyzes the reaction fraxetin+ NAD(P)H + 02= sideretin + NAD(P)(+) + H20. References: PMID:29581584 Sources: GOC:lr, RHEA:57844 Relationships: is a type of GO:0016709